{
  "gene": "UniProtKB:Q9NYQ8",
  "gene_symbol": "FAT2",
  "gene_name": "Protocadherin Fat 2",
  "term_id": "GO:0005886",
  "term_label": "plasma membrane"
}